antigen processing and presentation of polysaccharide antigen via MHC class II [GO:0002505] (biological process) References: PMID:16153240 Sources: GOC:add Regulation: regulated by regulation of antigen processing and presentation of polysaccharide antigen via MHC class II [GO:0002601]; negatively regulated by GO:0002602; positively regulated by GO:0002603 Also known as: polysaccharide antigen processing and presentation via MHC class II Definition: The process in which an antigen-presenting cell expresses a polysaccharide antigen on its cell surface in association with an MHC class II protein complex. Relationships: is a type of antigen processing and presentation of peptide or polysaccharide antigen via MHC class II [GO:0002504]